{
  "gene_symbol": "KIF25-AS1",
  "gene": "UniProtKB:Q9Y6Z4",
  "term_label": "Unknown biological process",
  "term_id": "UNKNOWN:0002",
  "gene_name": "Putative uncharacterized protein KIF25-AS1"
}